positive regulation of mitotic recombination-dependent replication fork processing [GO:0120292] (BP) References: PMID:23093942, PMID:28586299, PMID:31149897 Sources: GOC:krc, GOC:mah Also known as: positive regulation of recombination-dependent DNA replication, positive regulation of homologous recombination dependent replication fork recovery, positive regulation of mitotic recombination involved in replication fork processing Relationships: is_a positive regulation of DNA metabolic process [GO:0051054]; is a type of positive regulation of cell cycle process [GO:0090068]; is a type of regulation of mitotic recombination-dependent replication fork processing [GO:1903221]; positively regulates mitotic recombination-dependent replication fork processing [GO:1990426] Definition: Any process that activates or increases the frequency, rate or extent of mitotic recombination-dependent replication fork processing. Regulation of mitotic recombination prevents recombination between inappropriate homologous sequences. Proteins involved in homologous recombination are required for replication restart.